{
  "term_label": "embryonic organ development",
  "gene_name": "Transcriptional enhancer factor TEF-1",
  "term_id": "GO:0048568",
  "gene": "UniProtKB:P28347",
  "gene_symbol": "TEAD1"
}